{
  "gene": "UniProtKB:Q99426",
  "term_id": "GO:0051010",
  "gene_name": "Tubulin-folding cofactor B",
  "term_label": "microtubule plus-end binding",
  "gene_symbol": "TBCB"
}